Atg8-family conjugating enzyme activity [GO:0141046] (molecular function) Relationships: is a type of ubiquitin-like protein conjugating enzyme activity [GO:0061650] References: PMID:11100732, PMID:17986448, PMID:18704115, PMID:28234446, PMID:33909989 Also known as: E2, APG8 conjugating enzyme activity, Atg8-like conjugating activity, Atg8 conjugating enzyme activity Definition: Isoenergetic transfer of an Atg8 family modifier from one protein to a phosphatidylethanolamine or phosphatidylserine on a membrane, via the reaction X-Atg8 + Y = Y-Atg8 + X.